{
  "gene": "UniProtKB:Q96NJ1",
  "term_label": "Unknown cellular component",
  "gene_symbol": "Q96NJ1",
  "term_id": "UNKNOWN:0003",
  "gene_name": "Uncharacterized protein FLJ30774"
}